{
  "term_label": "syntaxin-1 binding",
  "term_id": "GO:0017075",
  "gene_name": "Synaptosomal-associated protein 25",
  "gene": "UniProtKB:P60880",
  "gene_symbol": "SNAP25"
}